{
  "term_id": "GO:0035845",
  "gene": "UniProtKB:P56715",
  "term_label": "photoreceptor cell outer segment organization",
  "gene_symbol": "RP1",
  "gene_name": "Oxygen-regulated protein 1"
}